nucleobase-containing compound kinase activity [GO:0019205] (molecular function) Also known as: nucleobase, nucleoside, nucleotide kinase activity Subtypes: nucleoside diphosphate kinase activity [GO:0004550], deoxynucleoside kinase activity [GO:0019136], nucleoside kinase activity [GO:0019206], nucleoside triphosphate adenylate kinase activity [GO:0046899], GO:0047507, nucleoside monophosphate kinase activity [GO:0050145], nucleoside phosphotransferase activity [GO:0050146], polynucleotide 5'-hydroxyl-kinase activity [GO:0051731], deoxynucleoside phosphate kinase activity, dGTP as phosphate donor [GO:0106367], deoxynucleoside phosphate kinase activity, dTTP as phosphate donor [GO:0106368], deoxynucleoside phosphate kinase activity, GTP as phosphate donor [GO:0106369] Relationships: is a type of GO:0016301 Definition: Catalysis of the transfer of a phosphate group, usually from ATP or GTP, to a nucleobase, nucleoside, nucleotide or polynucleotide substrate. Sources: GOC:jl